regulation of T-helper 2 cell differentiation [GO:0045628] (biological process) Definition: Any process that modulates the frequency, rate or extent of T-helper 2 cell differentiation. Sources: GOC:go_curators Also known as: regulation of T-helper 2 cell development Note: Note that immunologists typically use the word 'development' to refer to cells of B or T cell lineages undergoing the process that GO describes as 'cell differentiation'. Relationships: is a type of regulation of type 2 immune response [GO:0002828]; is a type of regulation of T-helper cell differentiation [GO:0045622]; regulates T-helper 2 cell differentiation [GO:0045064] Subtypes: GO:0045629, positive regulation of T-helper 2 cell differentiation [GO:0045630]